{
  "gene": "UniProtKB:P01111",
  "term_id": "GO:0003924",
  "gene_name": "GTPase NRas",
  "term_label": "GTPase activity",
  "gene_symbol": "NRAS"
}